cellular response to protozoan [GO:0099141] (biological process) Sources: GOC:dos Relationships: is a type of response to protozoan [GO:0001562] Definition: Any process that results in a change in state or activity of a cell (in terms of movement, secretion, enzyme production, gene expression, etc.) as a result of a stimulus from a protozoan.